{
  "term_label": "Unknown cellular component",
  "gene_name": "HCG2040265, isoform CRA_a",
  "term_id": "UNKNOWN:0003",
  "gene_symbol": "LOC730098",
  "gene": "UniProtKB:G3V523"
}